{
  "gene_name": "Mediator of RNA polymerase II transcription subunit 14",
  "term_label": "core mediator complex",
  "gene_symbol": "MED14",
  "gene": "UniProtKB:O60244",
  "term_id": "GO:0070847"
}